cadmium ion transmembrane transport [GO:0070574] (biological process) Definition: A process in which a cadmium ion is transported from one side of a membrane to the other by means of some agent such as a transporter or pore. Subtypes: GO:0036249 Relationships: is a type of cadmium ion transport [GO:0015691]; is a type of GO:0098655 Sources: GOC:mah Note: Note that this term is not intended for use in annotating lateral movement within membranes. Also known as: cadmium ion membrane transport, transmembrane cadmium transport